{
  "gene_name": "Beta-defensin 113",
  "gene": "UniProtKB:Q30KQ7",
  "term_id": "UNKNOWN:0002",
  "gene_symbol": "DEFB113",
  "term_label": "Unknown biological process"
}